{
  "term_id": "GO:0071222",
  "term_label": "cellular response to lipopolysaccharide",
  "gene_name": "T-lymphocyte activation antigen CD86",
  "gene_symbol": "CD86",
  "gene": "UniProtKB:P42081"
}